{
  "term_id": "GO:0005739",
  "term_label": "mitochondrion",
  "gene": "UniProtKB:P24752",
  "gene_symbol": "ACAT1",
  "gene_name": "Acetyl-CoA acetyltransferase, mitochondrial"
}